{
  "term_id": "GO:0032040",
  "term_label": "small-subunit processome",
  "gene": "UniProtKB:Q9BVI4",
  "gene_name": "Nucleolar complex protein 4 homolog",
  "gene_symbol": "NOC4L"
}